{
  "gene_symbol": "ZNF213",
  "gene": "UniProtKB:O14771",
  "term_id": "UNKNOWN:0003",
  "term_label": "Unknown cellular component",
  "gene_name": "Zinc finger protein 213"
}